positive regulation of mRNA modification [GO:0090366] (biological process) Sources: GOC:dph, GOC:sl, GOC:tb Relationships: is a type of GO:0090365; is a type of positive regulation of mRNA metabolic process [GO:1903313]; positively regulates mRNA modification [GO:0016556] Definition: Any process that increases the rate, frequency, or extent of the covalent alteration of one or more nucleotides within an mRNA molecule to produce an mRNA molecule with a sequence that differs from that coded genetically.